{
  "term_label": "mitochondrion",
  "term_id": "GO:0005739",
  "gene": "UniProtKB:Q8N490",
  "gene_name": "Probable hydrolase PNKD",
  "gene_symbol": "PNKD"
}